{
  "gene_symbol": "PHF20",
  "term_label": "NSL complex",
  "gene_name": "PHD finger protein 20",
  "gene": "UniProtKB:Q9BVI0",
  "term_id": "GO:0044545"
}